meiosis II cell cycle process [GO:0061983] (biological process) Relationships: is a type of meiotic cell cycle process [GO:1903046] Subtypes: meiosis II cytokinesis [GO:0007111], meiosis II [GO:0007135], metaphase/anaphase transition of meiosis II [GO:1990950] References: PMID:29385397 Definition: A process that coontributes to the second meiotic division. The second meiotic division separates chromatids resulting in a haploid number of chromosomes. Also known as: second meiotic division